peptidyl-proline 4-dioxygenase activity [GO:0031545] (molecular function) Sources: GOC:mah Definition: Catalysis of the reaction: peptidyl L-proline + 2-oxoglutarate + O2 = peptidyl trans-4-hydroxy-L-proline + succinate + CO2. Relationships: is a type of peptidyl-proline dioxygenase activity [GO:0031543] Subtypes: procollagen-proline 4-dioxygenase activity [GO:0004656], GO:0160082 Also known as: prolyl 4-hydroxylase, HIF-type prolyl 4-hydroxylase